intracellular nitrogen homeostasis [GO:0141067] (biological process) Subtypes: nitrogen utilization [GO:0019740] Also known as: cellular nitrogen homeostasis, nitrogen homeostasis Relationships: is a type of intracellular chemical homeostasis [GO:0055082] Sources: GOC:tb Definition: A homeostatic process involved in the maintenance of a steady state level of nitrogen within a cell.